{
  "term_id": "GO:0005886",
  "gene_name": "Short-wave-sensitive opsin 1",
  "gene_symbol": "OPN1SW",
  "term_label": "plasma membrane",
  "gene": "UniProtKB:P03999"
}